{
  "gene_symbol": "RNF25",
  "term_label": "ubiquitin-dependent protein catabolic process",
  "gene_name": "E3 ubiquitin-protein ligase RNF25",
  "term_id": "GO:0006511",
  "gene": "UniProtKB:Q96BH1"
}